{
  "term_id": "GO:0001755",
  "gene_symbol": "CORO1C",
  "gene": "UniProtKB:Q9ULV4",
  "gene_name": "Coronin-1C",
  "term_label": "neural crest cell migration"
}